{
  "term_id": "GO:0005737",
  "gene_name": "Small nuclear ribonucleoprotein-associated proteins B and B'",
  "gene_symbol": "SNRPB",
  "term_label": "cytoplasm",
  "gene": "UniProtKB:P14678"
}